Ecsit-NDUFAF1 complex [GO:0034985] (cellular component) Definition: Any large protein complex that contains Ecsit and NDUFAF1, is located in the mitochondrion, and is involved in the assembly of complex I of the oxidative phosphorylation system. In mammalian cells, three complexes of approximately 500, 600, and 850 kDa containing the 45 kDa isoform of Ecsit and NDUFAF1 have been observed. References: PMID:17344420 Relationships: is a type of mitochondrial protein-containing complex [GO:0098798]; is part of mitochondrial matrix [GO:0005759]